{
  "gene_symbol": "LCOR",
  "gene_name": "Ligand-dependent corepressor",
  "gene": "UniProtKB:Q96JN0",
  "term_label": "Unknown molecular function",
  "term_id": "UNKNOWN:0001"
}